{
  "term_label": "Unknown cellular component",
  "gene": "UniProtKB:E9PQ42",
  "term_id": "UNKNOWN:0003",
  "gene_symbol": "LOC84773-CYHR1",
  "gene_name": "TRAF-type domain-containing protein (Fragment)"
}